{
  "term_id": "UNKNOWN:0001",
  "gene_symbol": "ERVFC1-1",
  "term_label": "Unknown molecular function",
  "gene": "UniProtKB:P60608",
  "gene_name": "Endogenous retrovirus group FC1 member 1 Env polyprotein"
}